regulation of kinetochore assembly [GO:0090234] (biological process) Also known as: regulation of NMS complex assembly, regulation of chromosome-kinetochore attachment Definition: Any process that modulates the rate, frequency, or extent of kinetochore assembly, the aggregation, arrangement and bonding together of a set of components to form the kinetochore, a multisubunit complex that is located at the centromeric region of DNA and provides an attachment point for the spindle microtubules. Relationships: is a type of GO:0033044; is a type of regulation of protein-containing complex assembly [GO:0043254]; is a type of GO:1902115; regulates kinetochore assembly [GO:0051382] Sources: GOC:ascb_2009, GOC:dph, GOC:tb Subtypes: negative regulation of kinetochore assembly [GO:1905560], positive regulation of kinetochore assembly [GO:1905561]